accessory nerve formation [GO:0021608] (biological process) Sources: GOC:cls, GOC:dgh, GOC:dph, GOC:jid, GO_REF:0000021 Relationships: is a type of cranial nerve formation [GO:0021603]; is part of accessory nerve morphogenesis [GO:0021607] Also known as: CN XI biosynthesis, CN XI formation Definition: The process that gives rise to the accessory nerve. This process pertains to the initial formation of a structure from unspecified parts. The spinal branch of this motor nerve innervates the trapezius and the sternocleidomastoid muscles. The cranial branch joins the vagus nerve and innervates the same targets as the vagus nerve.